cardiolipin acyl-chain remodeling [GO:0035965] (BP) Relationships: is a type of cardiolipin metabolic process [GO:0032048] Also known as: cardiolipin maturation, cardiolipin acyl-chain remodelling, diphosphatidylglycerol remodeling Definition: Remodeling the acyl chains of premature (de novo synthesized) cardiolipin (1,3-bis(3-phosphatidyl)glycerol), through sequential deacylation and re-acylation reactions, to generate mature cardiolipin containing high-levels of unsaturated fatty acids. References: PMID:19244244 Sources: GOC:bf, GOC:rb